{
  "gene_name": "Coagulation factor XI",
  "gene": "UniProtKB:P03951",
  "gene_symbol": "F11",
  "term_id": "GO:0031639",
  "term_label": "plasminogen activation"
}